{
  "gene_name": "FYVE, RhoGEF and PH domain-containing protein 1",
  "term_id": "GO:0046847",
  "gene": "UniProtKB:P98174",
  "term_label": "filopodium assembly",
  "gene_symbol": "FGD1"
}